{
  "term_id": "GO:0005886",
  "term_label": "plasma membrane",
  "gene_name": "XK-related protein 7",
  "gene_symbol": "XKR7",
  "gene": "UniProtKB:Q5GH72"
}